{
  "gene_name": "ADP-ribosylation factor 4",
  "term_id": "GO:0005525",
  "term_label": "GTP binding",
  "gene": "UniProtKB:P18085",
  "gene_symbol": "ARF4"
}